{
  "gene_name": "Plasma membrane calcium-transporting ATPase 4",
  "term_label": "plasma membrane",
  "term_id": "GO:0005886",
  "gene_symbol": "ATP2B4",
  "gene": "UniProtKB:P23634"
}